{
  "gene_symbol": "HLA-DQB2",
  "gene_name": "HLA class II histocompatibility antigen, DQ beta 2 chain",
  "gene": "UniProtKB:P05538",
  "term_label": "lysosomal membrane",
  "term_id": "GO:0005765"
}